{
  "term_label": "microtubule cytoskeleton organization",
  "gene_name": "Microtubule-associated protein 1S",
  "term_id": "GO:0000226",
  "gene_symbol": "MAP1S",
  "gene": "UniProtKB:Q66K74"
}